leukocyte activation-dependent arrest [GO:0050903] (biological process) References: PMID:14680625, PMID:14708592, PMID:7507411, PMID:8600538 Sources: ISBN:0781735149 Definition: The formation of an integrin-dependent strong adhesive bond between leukocytes and blood vessel endothelial cells which is dependent on prior activation of the leukocyte and leads to the firm attachment of the leukocyte to the endothelial surface, typically the third step in cellular extravasation. Relationships: is a type of GO:0061756; is part of cellular extravasation [GO:0045123]